{
  "term_label": "plasma membrane",
  "term_id": "GO:0005886",
  "gene": "UniProtKB:P10301",
  "gene_symbol": "RRAS",
  "gene_name": "Ras-related protein R-Ras"
}